histone ubiquitin ligase activity [GO:0140852] (molecular function) Definition: Catalysis of the transfer of ubiquitin to a histone substrate. Sources: GOC:curators Subtypes: histone H2A ubiquitin ligase activity [GO:0141053], histone H2B ubiquitin ligase activity [GO:0141054], GO:0141055, histone H4 ubiquitin ligase activity [GO:0141056] Relationships: is a type of ubiquitin protein ligase activity [GO:0061630]; is a type of histone modifying activity [GO:0140993]